insulin secretion involved in cellular response to glucose stimulus [GO:0035773] (biological process) Definition: The regulated release of proinsulin from secretory granules (B granules) in the B cells of the pancreas; accompanied by cleavage of proinsulin to form mature insulin, in response to a glucose stimulus. References: PMID:8492079 Sources: GOC:bf, GOC:yaf Also known as: insulin secretion involved in cellular response to glucose Relationships: is a type of insulin secretion [GO:0030073]; is a type of establishment of localization in cell [GO:0051649]; is part of cellular response to glucose stimulus [GO:0071333] Regulation: positively regulated by positive regulation of insulin secretion involved in cellular response to glucose stimulus [GO:0035774]; regulated by regulation of insulin secretion involved in cellular response to glucose stimulus [GO:0061178]; negatively regulated by negative regulation of insulin secretion involved in cellular response to glucose stimulus [GO:0061179]